response to benzoic acid [GO:0080021] (biological process) Relationships: is a type of GO:1901700 Also known as: response to benzoic acid stimulus References: PMID:18753285 Subtypes: GO:0071319 Definition: Any process that results in a change in state or activity of a cell or an organism (in terms of movement, secretion, enzyme production, gene expression, etc.) as a result of a benzoic acid stimulus.